{
  "gene_symbol": "ALDH2",
  "term_id": "GO:0005739",
  "gene_name": "Aldehyde dehydrogenase, mitochondrial",
  "term_label": "mitochondrion",
  "gene": "UniProtKB:P05091"
}